{
  "term_id": "UNKNOWN:0003",
  "term_label": "Unknown cellular component",
  "gene_name": "Uncharacterized protein",
  "gene": "UniProtKB:A0A6Q8PFQ6",
  "gene_symbol": "A0A6Q8PFQ6"
}